{
  "term_id": "GO:0003924",
  "gene_name": "Ras-related protein Rab-11A",
  "gene_symbol": "RAB11A",
  "term_label": "GTPase activity",
  "gene": "UniProtKB:P62491"
}